{
  "gene_name": "Ubiquitin-like modifier-activating enzyme ATG7",
  "term_id": "GO:0034727",
  "gene_symbol": "ATG7",
  "term_label": "piecemeal microautophagy of the nucleus",
  "gene": "UniProtKB:O95352"
}